{
  "term_label": "N6-methyladenosine-containing RNA reader activity",
  "gene_name": "YTH domain-containing family protein 3",
  "gene_symbol": "YTHDF3",
  "term_id": "GO:1990247",
  "gene": "UniProtKB:Q7Z739"
}